maintenance of nucleus location [GO:0051658] (biological process) Also known as: maintenance of cell nucleus location, maintenance of nucleus localization Relationships: is a type of nucleus localization [GO:0051647]; is a type of maintenance of organelle location [GO:0051657] Definition: Any process in which the nucleus is maintained in a specific location within a cell and prevented from moving elsewhere. Subtypes: maintenance of oocyte nucleus location involved in oocyte dorsal/ventral axis specification [GO:0042070] Sources: GOC:ai, GOC:dph, GOC:tb